{
  "gene": "UniProtKB:Q06413",
  "gene_name": "Myocyte-specific enhancer factor 2C",
  "term_id": "GO:0007507",
  "gene_symbol": "MEF2C",
  "term_label": "heart development"
}